{
  "term_id": "GO:0003870",
  "term_label": "5-aminolevulinate synthase activity",
  "gene_symbol": "ALAS1",
  "gene": "UniProtKB:P13196",
  "gene_name": "5-aminolevulinate synthase, non-specific, mitochondrial"
}